{
  "term_id": "GO:0003723",
  "gene_name": "Exosome complex component RRP41",
  "term_label": "RNA binding",
  "gene": "UniProtKB:Q9NPD3",
  "gene_symbol": "EXOSC4"
}